{
  "gene": "UniProtKB:P36955",
  "term_id": "GO:0005615",
  "gene_name": "Pigment epithelium-derived factor",
  "gene_symbol": "SERPINF1",
  "term_label": "extracellular space"
}